{
  "term_label": "cytoplasm",
  "gene_symbol": "ARHGAP9",
  "term_id": "GO:0005737",
  "gene_name": "Rho GTPase-activating protein 9",
  "gene": "UniProtKB:Q9BRR9"
}